{
  "gene_symbol": "IGSF9",
  "term_id": "GO:0030424",
  "gene": "UniProtKB:Q9P2J2",
  "gene_name": "Protein turtle homolog A",
  "term_label": "axon"
}